RecFOR complex [GO:0043850] (cellular component) References: PMID:12769856 Definition: A heterotrimeric complex composed of the subunits RecF, RecO and RecR. Mediates the loading of RecA protein specifically onto SSB-coated gapped DNA during DNA repair. Relationships: is a type of protein-containing complex [GO:0032991]; is part of GO:0005694